regulation of signal transduction by p53 class mediator [GO:1901796] (biological process) Subtypes: regulation of DNA damage response, signal transduction by p53 class mediator [GO:0043516], negative regulation of signal transduction by p53 class mediator [GO:1901797], positive regulation of signal transduction by p53 class mediator [GO:1901798], regulation of intrinsic apoptotic signaling pathway by p53 class mediator [GO:1902253] Definition: Any process that modulates the frequency, rate or extent of signal transduction by p53 class mediator. Sources: GOC:TermGenie Relationships: is a type of regulation of intracellular signal transduction [GO:1902531]; regulates GO:0072331